phlorizin hydrolase activity [GO:0140749] (molecular function) References: PMID:9762914 Sources: RHEA:69639 Relationships: is a type of GO:0004553 Definition: Catalysis of the reaction: phlorizin + H2O = beta-D-glucose + phloretin.